response to ultrasound [GO:1990478] (biological process) Definition: Any process that results in a change in state or activity of a cell or an organism (in terms of movement, secretion, enzyme production, gene expression, etc.) as a result of an ultrasonic stimulus. References: PMID:20950932 Relationships: is a type of response to mechanical stimulus [GO:0009612]